{
  "gene_name": "Syntaxin-binding protein 2",
  "gene_symbol": "STXBP2",
  "gene": "UniProtKB:Q15833",
  "term_label": "syntaxin-1 binding",
  "term_id": "GO:0017075"
}